{
  "gene_symbol": "TMEM114",
  "gene_name": "Transmembrane protein 114",
  "term_id": "GO:0016324",
  "term_label": "apical plasma membrane",
  "gene": "UniProtKB:B3SHH9"
}